{
  "term_label": "protein ubiquitination",
  "gene": "UniProtKB:Q8WW12",
  "gene_name": "PEST proteolytic signal-containing nuclear protein",
  "term_id": "GO:0016567",
  "gene_symbol": "PCNP"
}